{
  "term_label": "sphingosine-1-phosphate receptor activity",
  "gene": "UniProtKB:O95136",
  "gene_symbol": "S1PR2",
  "gene_name": "Sphingosine 1-phosphate receptor 2",
  "term_id": "GO:0038036"
}